plasmatocyte differentiation [GO:0042387] (biological process) Regulation: regulated by GO:0045613; negatively regulated by negative regulation of plasmatocyte differentiation [GO:0045614]; positively regulated by positive regulation of plasmatocyte differentiation [GO:0045615] Definition: The process in which a hemocyte precursor cell acquires the characteristics of the phagocytic blood-cell type, the plasmatocyte. Plasmatocytes are a class of arthropod hemocytes important in the cellular defense response. Relationships: is a type of hemocyte differentiation [GO:0042386] Subtypes: embryonic plasmatocyte differentiation [GO:0035164], GO:0035169 References: PMID:11921077, PMID:8174791